{
  "term_id": "GO:0002323",
  "gene": "UniProtKB:P01567",
  "gene_symbol": "IFNA7",
  "term_label": "natural killer cell activation involved in immune response",
  "gene_name": "Interferon alpha-7"
}